{
  "gene": "UniProtKB:P15509",
  "term_id": "GO:0070195",
  "gene_symbol": "CSF2RA",
  "gene_name": "Granulocyte-macrophage colony-stimulating factor receptor subunit alpha",
  "term_label": "growth hormone receptor complex"
}